{
  "term_label": "autophagosome-lysosome fusion",
  "term_id": "GO:0061909",
  "gene_symbol": "ATP13A2",
  "gene_name": "Polyamine-transporting ATPase 13A2",
  "gene": "UniProtKB:Q9NQ11"
}